{
  "term_id": "GO:0032809",
  "gene": "UniProtKB:Q14003",
  "gene_symbol": "KCNC3",
  "gene_name": "Potassium voltage-gated channel subfamily C member 3",
  "term_label": "neuronal cell body membrane"
}